{
  "gene_symbol": "CORO1B",
  "term_id": "GO:0051015",
  "term_label": "actin filament binding",
  "gene_name": "Coronin-1B",
  "gene": "UniProtKB:Q9BR76"
}